{
  "gene": "UniProtKB:P12724",
  "gene_symbol": "RNASE3",
  "gene_name": "Eosinophil cationic protein",
  "term_label": "extracellular space",
  "term_id": "GO:0005615"
}